vanillin catabolic process [GO:0042190] (biological process) Relationships: is a type of vanillin metabolic process [GO:0018982]; is a type of phenol-containing compound catabolic process [GO:0019336]; is_a aldehyde catabolic process [GO:0046185]; is a type of ether catabolic process [GO:1901502] Also known as: vanillic aldehyde catabolic process, vanillic aldehyde catabolism, vanillin breakdown, vanillin catabolism, vanillin degradation Definition: The chemical reactions and pathways resulting in the breakdown of vanillin, an aromatic hydrocarbon which occurs naturally in black vanilla bean pods. Sources: GOC:jl